{
  "term_label": "Golgi apparatus",
  "gene": "UniProtKB:Q9NV96",
  "gene_name": "Cell cycle control protein 50A",
  "term_id": "GO:0005794",
  "gene_symbol": "TMEM30A"
}